{
  "term_id": "GO:0086012",
  "gene": "UniProtKB:O60939",
  "gene_name": "Sodium channel subunit beta-2",
  "gene_symbol": "SCN2B",
  "term_label": "membrane depolarization during cardiac muscle cell action potential"
}